mitochondrial inner-outer membrane contact site [GO:0044289] (cellular component) Also known as: contact site, bridge contact site References: PMID:22009199 Relationships: is a type of GO:0044232; is part of GO:0031966 Definition: Sites of close apposition of the inner and outer mitochondrial membrane.